{
  "gene_symbol": "SHOX2",
  "gene": "UniProtKB:O60902",
  "term_id": "GO:0005634",
  "gene_name": "Short stature homeobox protein 2",
  "term_label": "nucleus"
}